positive regulation of antigen processing and presentation of endogenous peptide antigen via MHC class I [GO:1904284] (biological process) Definition: Any process that activates or increases the frequency, rate or extent of antigen processing and presentation of endogenous peptide antigen via MHC class I. Relationships: is a type of GO:0002591; is a type of regulation of antigen processing and presentation of endogenous peptide antigen via MHC class I [GO:1904282]; positively regulates GO:0019885 Also known as: positive regulation of endogenous peptide antigen processing and presentation via MHC class I, up regulation of antigen processing and presentation of endogenous peptide antigen via MHC class I, up regulation of endogenous peptide antigen processing and presentation via MHC class I, up-regulation of antigen processing and presentation of endogenous peptide antigen via MHC class I, up-regulation of endogenous peptide antigen processing and presentation via MHC class I, upregulation of antigen processing and presentation of endogenous peptide antigen via MHC class I, upregulation of endogenous peptide antigen processing and presentation via MHC class I, activation of antigen processing and presentation of endogenous peptide antigen via MHC class I, activation of endogenous peptide antigen processing and presentation via MHC class I References: PMID:24643698 Sources: GOC:BHF, GOC:TermGenie, GOC:rl, GO_REF:0000058